{
  "term_label": "Unknown cellular component",
  "gene_name": "Putative inactive cytochrome P450 family member 4Z2",
  "term_id": "UNKNOWN:0003",
  "gene": "UniProtKB:Q8N1L4",
  "gene_symbol": "CYP4Z2P"
}